{
  "gene": "UniProtKB:Q13009",
  "term_id": "GO:0045202",
  "gene_symbol": "TIAM1",
  "gene_name": "Rho guanine nucleotide exchange factor TIAM1",
  "term_label": "synapse"
}